{
  "term_label": "phospholipase C-activating serotonin receptor signaling pathway",
  "gene": "UniProtKB:P28335",
  "gene_name": "5-hydroxytryptamine receptor 2C",
  "term_id": "GO:0007208",
  "gene_symbol": "HTR2C"
}